regulation of adenosine transport [GO:0032249] (biological process) Relationships: is_a regulation of purine nucleoside transport [GO:0032245]; regulates adenosine transport [GO:0032238] Definition: Any process that modulates the frequency, rate or extent of the directed movement of adenosine into, out of or within a cell, or between cells, by means of some agent such as a transporter or pore. Sources: GOC:mah Subtypes: negative regulation of adenosine transport [GO:0032250], positive regulation of adenosine transport [GO:0032251]